{
  "gene_name": "PR domain zinc finger protein 14",
  "term_label": "RNA polymerase II transcription regulatory region sequence-specific DNA binding",
  "gene": "UniProtKB:Q9GZV8",
  "term_id": "GO:0000977",
  "gene_symbol": "PRDM14"
}